single-strand selective uracil DNA N-glycosylase activity [GO:0017065] (molecular function) Definition: Catalysis of the cleavage of the N-C1' glycosidic bond between the damaged DNA base and the deoxyribose sugar, releasing a free base and leaving an apyrimidinic (AP) site. Enzymes with this activity recognize and remove uracil bases present in single-stranded DNA. Also known as: single-strand selective monofunctional uracil-DNA glycosylase activity Relationships: is a type of uracil DNA N-glycosylase activity [GO:0004844] References: PMID:9224623 Sources: GOC:elh